detection of hypoxic conditions in blood by aortic body chemoreceptor signaling [GO:0003033] (biological process) Definition: The process in which information about a lack of oxygen are received and are converted to a molecular signal by chemoreceptors in the aortic bodies. Relationships: is a type of detection of hypoxic conditions in blood by chemoreceptor signaling [GO:0002007]; is part of regulation of systemic arterial blood pressure by aortic body chemoreceptor signaling [GO:0003028] Sources: GOC:mtg_cardio Also known as: detection of hypoxic conditions in blood by aortic body chemoreceptor signalling